{
  "gene_name": "WD repeat-containing protein 87",
  "gene_symbol": "WDR87",
  "term_id": "UNKNOWN:0001",
  "term_label": "Unknown molecular function",
  "gene": "UniProtKB:Q6ZQQ6"
}